{
  "gene_name": "Lactase_phlorizin hydrolase",
  "term_label": "beta-glucosidase activity",
  "gene": "UniProtKB:P09848",
  "term_id": "GO:0008422",
  "gene_symbol": "LCT"
}